{
  "gene_symbol": "SLC25A20",
  "term_id": "GO:0006839",
  "gene": "UniProtKB:O43772",
  "gene_name": "Mitochondrial carnitine_acylcarnitine carrier protein",
  "term_label": "mitochondrial transport"
}